ATR-ATRIP complex [GO:0070310] (cellular component) Relationships: is a type of nuclear protein-containing complex [GO:0140513] Also known as: Mec1-Lcd1 complex, Rad3-Rad26 complex References: PMID:14724280 Sources: GOC:mah Definition: A protein complex that contains the protein kinase ATR and ATR-interacting protein (ATRIP) and binds single-stranded DNA; ssDNA binding affinity is increased in the presence of replication protein A.